{
  "term_label": "response to exogenous dsRNA",
  "gene": "UniProtKB:P01563",
  "gene_name": "Interferon alpha-2",
  "gene_symbol": "IFNA2",
  "term_id": "GO:0043330"
}